{
  "gene_symbol": "CYP2S1",
  "term_label": "cytoplasm",
  "gene_name": "Cytochrome P450 2S1",
  "term_id": "GO:0005737",
  "gene": "UniProtKB:Q96SQ9"
}